{
  "term_id": "GO:0030334",
  "gene": "UniProtKB:Q4VCS5",
  "term_label": "regulation of cell migration",
  "gene_name": "Angiomotin",
  "gene_symbol": "AMOT"
}